{
  "term_id": "GO:0061630",
  "gene": "UniProtKB:Q9Y252",
  "gene_name": "E3 ubiquitin-protein ligase RNF6",
  "term_label": "ubiquitin protein ligase activity",
  "gene_symbol": "RNF6"
}